response to photooxidative stress [GO:0080183] (biological process) Relationships: is_a response to oxidative stress [GO:0006979] Definition: Any process that results in a change in state or activity of a cell or organism (in terms of movement, secretion, enzyme production, gene expression, etc.) as the result of a photooxidative stress, the light-dependent generation of active oxygen species. The process begins with detection of the stimulus and ends with a change in state or activity or the cell or organism. Sources: DOI:10.1111/j.1399-3054.1994.tb03042.x